{
  "gene_name": "DALR anticodon-binding domain-containing protein 3",
  "term_label": "tRNA binding",
  "gene": "UniProtKB:Q5D0E6",
  "term_id": "GO:0000049",
  "gene_symbol": "DALRD3"
}